{
  "gene_symbol": "FOXJ1",
  "gene_name": "Forkhead box protein J1",
  "gene": "UniProtKB:Q92949",
  "term_label": "DNA-binding transcription factor activity, RNA polymerase II-specific",
  "term_id": "GO:0000981"
}